negative regulation of orcinol biosynthetic process [GO:1900702] (biological process) Relationships: is a type of negative regulation of secondary metabolite biosynthetic process [GO:1900377]; is a type of regulation of orcinol biosynthetic process [GO:1900701]; negatively regulates orcinol biosynthetic process [GO:0046197] Sources: GOC:TermGenie, GOC:di Definition: Any process that stops, prevents or reduces the frequency, rate or extent of orcinol biosynthetic process. Also known as: down regulation of orcinol anabolism, down regulation of orcinol biosynthesis, down regulation of orcinol biosynthetic process, down regulation of orcinol formation, down regulation of orcinol synthesis, down-regulation of orcinol anabolism, down-regulation of orcinol biosynthesis, down-regulation of orcinol biosynthetic process, down-regulation of orcinol formation, down-regulation of orcinol synthesis, downregulation of orcinol anabolism, downregulation of orcinol biosynthesis, downregulation of orcinol biosynthetic process, downregulation of orcinol formation, downregulation of orcinol synthesis, inhibition of orcinol anabolism, inhibition of orcinol biosynthesis, inhibition of orcinol formation, inhibition of orcinol synthesis, negative regulation of orcinol anabolism, negative regulation of orcinol biosynthesis, negative regulation of orcinol formation, negative regulation of orcinol synthesis, inhibition of orcinol biosynthetic process